{
  "gene_symbol": "XKRY",
  "gene_name": "Testis-specific XK-related protein, Y-linked",
  "gene": "UniProtKB:O14609",
  "term_label": "Unknown biological process",
  "term_id": "UNKNOWN:0002"
}